chemokine (C-C motif) ligand 5 signaling pathway [GO:0035689] (biological process) Also known as: CCL5-mediated signaling pathway, RANTES-mediated signaling pathway, chemokine (C-C motif) ligand 5 signalling pathway Relationships: is a type of chemokine-mediated signaling pathway [GO:0070098] References: PMID:18337562 Sources: GOC:BHF Definition: The series of molecular signals initiated by chemokine CCL5 binding to its receptor on the surface of a target cell, and ending with the regulation of a downstream cellular process, e.g. transcription.